{
  "term_id": "GO:0045065",
  "gene": "UniProtKB:P01732",
  "gene_symbol": "CD8A",
  "gene_name": "T-cell surface glycoprotein CD8 alpha chain",
  "term_label": "cytotoxic T cell differentiation"
}